{
  "gene_name": "Myotubularin-related protein 14",
  "gene_symbol": "MTMR14",
  "term_label": "phosphatidylinositol-3-phosphate phosphatase activity",
  "term_id": "GO:0004438",
  "gene": "UniProtKB:Q8NCE2"
}